ferric triacetylfusarinine C import into cell [GO:0015686] (biological process) Also known as: ferric triacetylfusarinine C transport Definition: The directed movement of ferric triacetylfusarinine C into, out of or within a cell, or between cells, by means of some agent such as a transporter or pore. Relationships: is a type of siderophore-iron import into cell [GO:0033214]; is a type of nitrogen compound transport [GO:0071705] Sources: GOC:ai